{
  "term_label": "Unknown cellular component",
  "gene_symbol": "STARD13",
  "gene_name": "StAR-related lipid transfer protein 13",
  "gene": "UniProtKB:Q9Y3M8",
  "term_id": "UNKNOWN:0003"
}